{
  "gene_name": "N-glycosylase_DNA lyase",
  "gene_symbol": "OGG1",
  "term_label": "8-oxo-7,8-dihydroguanine DNA N-glycosylase activity",
  "gene": "UniProtKB:O15527",
  "term_id": "GO:0034039"
}